{
  "gene_symbol": "GTF2I",
  "term_id": "GO:0005634",
  "gene_name": "General transcription factor II-I",
  "term_label": "nucleus",
  "gene": "UniProtKB:P78347"
}